{
  "term_label": "Ndc80 complex",
  "gene_symbol": "NDC80",
  "gene_name": "Kinetochore protein NDC80 homolog",
  "term_id": "GO:0031262",
  "gene": "UniProtKB:O14777"
}